pyrogallol hydroxytransferase activity [GO:0018706] (molecular function) Also known as: pyrogallol hydroxyltransferase activity, 1,2,3,5-tetrahydroxybenzene hydroxyltransferase activity, 1,2,3,5-tetrahydroxybenzene-pyrogallol hydroxyltransferase (transhydroxylase), 1,2,3,5-tetrahydroxybenzene:1,2,3-trihydroxybenzene hydroxyltransferase activity, 1,2,3,5-tetrahydroxybenzene:1,2,3-trihydroxybenzene hydroxytransferase activity, 1,2,3,5-tetrahydroxybenzene:pyrogallol transhydroxylase activity, transhydroxylase activity Sources: RHEA:21000 Relationships: is a type of oxidoreductase activity [GO:0016491] Definition: Catalysis of the reaction: 1,2,3,5-tetrahydroxybenzene + 1,2,3-trihydroxybenzene = 1,3,5-trihydroxybenzene + 1,2,3,5-tetrahydroxybenzene.